{
  "term_label": "olfactory receptor activity",
  "term_id": "GO:0004984",
  "gene_name": "Olfactory receptor 5T2",
  "gene_symbol": "OR5T2",
  "gene": "UniProtKB:Q8NGG2"
}